protein N-terminal-serine acetyltransferase activity [GO:1990189] (molecular function) Also known as: peptide-serine-alpha-N-acetyltransferase activity References: PMID:23912279 Sources: RHEA:50504 Definition: Catalysis of the reaction: acetyl-CoA + N-terminal L-seryl-[protein] = CoA + H+ + N-terminal Nalpha-acetyl-L-seryl-[protein]. Relationships: is_a protein-N-terminal amino-acid acetyltransferase activity [GO:0004596]